{
  "gene_symbol": "MCCC2",
  "term_label": "L-leucine catabolic process",
  "gene": "UniProtKB:Q9HCC0",
  "gene_name": "Methylcrotonoyl-CoA carboxylase beta chain, mitochondrial",
  "term_id": "GO:0006552"
}